cytolytic granule lumen [GO:1904856] (cellular component) Definition: Any cytoplasmic membrane-bounded vesicle lumen that is part of a cytolytic granule. Relationships: is a type of vacuolar lumen [GO:0005775]; is a type of cytoplasmic vesicle lumen [GO:0060205]; is part of cytolytic granule [GO:0044194] References: PMID:17272266, PMID:21247065 Sources: GOC:TermGenie, GO_REF:0000064 Also known as: cytolytic granule cytoplasmic membrane-bounded vesicle lumen, cytoplasmic membrane-bounded vesicle lumen of cytolytic granule, cytoplasmic membrane-enclosed vesicle lumen of cytolytic granule